{
  "term_label": "carbohydrate homeostasis",
  "term_id": "GO:0033500",
  "gene_symbol": "VGF",
  "gene": "UniProtKB:O15240",
  "gene_name": "Neurosecretory protein VGF"
}